{
  "gene": "UniProtKB:P01210",
  "term_id": "GO:0007600",
  "gene_symbol": "PENK",
  "gene_name": "Proenkephalin-A",
  "term_label": "sensory perception"
}